regulation of pheromone response MAPK cascade [GO:0180039] (biological process) Subtypes: positive regulation of pheromone response MAPK cascade [GO:0062038], negative regulation of pheromone response MAPK cascade [GO:0180040] Sources: GOC:vw Relationships: is_a regulation of MAPK cascade [GO:0043408]; regulates pheromone response MAPK cascade [GO:0071507] Definition: Any process that modulates the frequency, rate or extent of a pheromone response MAPK cascade.